{
  "term_label": "Unknown biological process",
  "gene_name": "Putative uncharacterized protein encoded by MIR1915-HG",
  "gene": "UniProtKB:Q5T4H9",
  "term_id": "UNKNOWN:0002",
  "gene_symbol": "MIR1915HG"
}